high-affinity D-glucose transmembrane transporter activity [GO:0140108] (molecular function) Definition: Enables the transfer of D-glucose from one side of a membrane to the other. In high-affinity transport the transporter is able to bind the solute even if it is only present at very low concentrations. References: PMID:25411338 Relationships: is a type of D-glucose transmembrane transporter activity [GO:0055056] Also known as: high-affinity glucose transmembrane transporter activity